sucrose 1F-fructosyltransferase activity [GO:0050306] (molecular function) Sources: EC:2.4.1.99 Also known as: SST activity, sucrose 1(F)-fructosyltransferase activity, sucrose-sucrose 1-fructosyltransferase activity, sucrose:sucrose 1'-beta-D-fructosyltransferase activity, sucrose:sucrose 1(F)-beta-D-fructosyltransferase activity, sucrose:sucrose 1-fructosyltransferase activity, sucrose:sucrose 1F-beta-D-fructosyltransferase activity, sucrose:sucrose fructosyltransferase activity Definition: Catalysis of the reaction: 2 sucrose = D-glucose + 1F-beta-D-fructosylsucrose. Relationships: is a type of fructosyltransferase activity [GO:0050738]